type 1B serotonin receptor binding [GO:0031822] (MF) Relationships: is a type of G protein-coupled serotonin receptor binding [GO:0031821] Definition: Binding to a type 1B serotonin receptor. Also known as: 5-hydroxytryptamine 1B receptor binding, type 1B serotonin receptor ligand Sources: GOC:mah, GOC:nln